phosphoglycerate transmembrane transport [GO:0015713] (biological process) Definition: The process in which phosphoglycerate is transported across a lipid bilayer, from one side of a membrane to the other. Also known as: phosphoglycerate transport Relationships: is a type of GO:0042873 Sources: GOC:krc